{
  "gene": "UniProtKB:Q9UJ42",
  "gene_symbol": "GPR160",
  "gene_name": "Probable G-protein coupled receptor 160",
  "term_id": "UNKNOWN:0002",
  "term_label": "Unknown biological process"
}